{
  "term_id": "GO:0004364",
  "gene_name": "Glutathione S-transferase omega-1",
  "gene": "UniProtKB:P78417",
  "gene_symbol": "GSTO1",
  "term_label": "glutathione transferase activity"
}